{
  "term_label": "tRNA processing",
  "gene_symbol": "RPP30",
  "gene_name": "Ribonuclease P protein subunit p30",
  "gene": "UniProtKB:P78346",
  "term_id": "GO:0008033"
}